(1->3)-beta-D-glucan metabolic process [GO:0006074] (biological process) Sources: ISBN:0198506732 Also known as: 1,3-beta-D-glucan metabolic process, 1,3-beta-glucan metabolic process, 1,3-beta-D-glucan metabolism, beta-1,3 glucan metabolic process, beta-1,3 glucan metabolism Subtypes: (1->3)-beta-D-glucan biosynthetic process [GO:0006075], (1->3)-beta-D-glucan catabolic process [GO:0006076], cell wall (1->3)-beta-D-glucan metabolic process [GO:0034407] Definition: The chemical reactions and pathways involving (1->3)-beta-D-glucans, compounds composed of glucose residues linked by (1->3)-beta-D-glucosidic bonds. Relationships: is a type of beta-glucan metabolic process [GO:0051273]